{
  "gene_name": "Cholesterol 25-hydroxylase",
  "gene": "UniProtKB:O95992",
  "gene_symbol": "CH25H",
  "term_id": "GO:0016126",
  "term_label": "sterol biosynthetic process"
}